{
  "term_id": "GO:0005891",
  "gene": "UniProtKB:Q08289",
  "gene_symbol": "CACNB2",
  "gene_name": "Voltage-dependent L-type calcium channel subunit beta-2",
  "term_label": "voltage-gated calcium channel complex"
}